{
  "term_label": "intracellular signal transduction",
  "gene": "UniProtKB:Q96CX6",
  "gene_name": "Leucine-rich repeat-containing protein 58",
  "gene_symbol": "LRRC58",
  "term_id": "GO:0035556"
}